regulation of systemic arterial blood pressure by circulatory epinephrine-norepinephrine [GO:0003101] (biological process) Also known as: regulation of blood pressure by circulating adrenaline-noradrenaline Definition: The process in which epinephrine-norepinephrine modulate the force with which blood passes through the circulatory system. Sources: GOC:mtg_cardio Relationships: is a type of regulation of systemic arterial blood pressure by hormone [GO:0001990]